{
  "gene": "UniProtKB:Q5VVC0",
  "term_id": "GO:0007130",
  "term_label": "synaptonemal complex assembly",
  "gene_symbol": "SPO16",
  "gene_name": "Protein SPO16 homolog"
}